{
  "gene": "UniProtKB:P52948",
  "term_id": "GO:0003723",
  "gene_name": "Nuclear pore complex protein Nup98-Nup96",
  "gene_symbol": "NUP98",
  "term_label": "RNA binding"
}